{
  "term_label": "cerebral cortex development",
  "gene": "UniProtKB:Q15058",
  "gene_name": "Kinesin-like protein KIF14",
  "gene_symbol": "KIF14",
  "term_id": "GO:0021987"
}